{
  "term_id": "UNKNOWN:0003",
  "term_label": "Unknown cellular component",
  "gene_name": "Gasdermin-B",
  "gene_symbol": "GSDMB",
  "gene": "UniProtKB:Q8TAX9"
}